{
  "gene": "UniProtKB:Q96RJ3",
  "term_id": "GO:0030890",
  "gene_symbol": "TNFRSF13C",
  "gene_name": "Tumor necrosis factor receptor superfamily member 13C",
  "term_label": "positive regulation of B cell proliferation"
}